{
  "term_label": "cell chemotaxis",
  "gene": "UniProtKB:P51677",
  "term_id": "GO:0060326",
  "gene_name": "C-C chemokine receptor type 3",
  "gene_symbol": "CCR3"
}